{
  "gene_symbol": "ABLIM2",
  "term_id": "GO:0015629",
  "gene": "UniProtKB:Q6H8Q1",
  "term_label": "actin cytoskeleton",
  "gene_name": "Actin-binding LIM protein 2"
}